glycoprotein transport [GO:0034436] (biological process) Definition: The directed movement of a glycoprotein, a protein that contains covalently bound glycose (i.e. monosaccharide) residues, into, out of or within a cell, or between cells, by means of some agent such as a transporter or pore. Sources: GOC:BHF, GOC:mah, GOC:rl Relationships: is a type of protein transport [GO:0015031]; is_a carbohydrate derivative transport [GO:1901264]